{
  "gene_symbol": "SLC6A11",
  "gene": "UniProtKB:P48066",
  "gene_name": "Sodium- and chloride-dependent GABA transporter 3",
  "term_id": "GO:0005886",
  "term_label": "plasma membrane"
}